{
  "gene_name": "Potassium channel subfamily K member 5",
  "term_id": "GO:0015271",
  "gene": "UniProtKB:O95279",
  "gene_symbol": "KCNK5",
  "term_label": "outward rectifier potassium channel activity"
}